{
  "term_label": "ubiquitin protein ligase activity",
  "term_id": "GO:0061630",
  "gene": "UniProtKB:O76050",
  "gene_name": "E3 ubiquitin-protein ligase NEURL1",
  "gene_symbol": "NEURL1"
}